{
  "term_id": "GO:0010485",
  "gene": "UniProtKB:O95251",
  "term_label": "histone H4 acetyltransferase activity",
  "gene_symbol": "KAT7",
  "gene_name": "Histone acetyltransferase KAT7"
}